{
  "term_label": "cytoplasm",
  "term_id": "GO:0005737",
  "gene": "UniProtKB:P20794",
  "gene_symbol": "MAK",
  "gene_name": "Serine_threonine-protein kinase MAK"
}